{
  "gene_symbol": "ARHGEF10L",
  "term_label": "cytoplasm",
  "gene_name": "Rho guanine nucleotide exchange factor 10-like protein",
  "gene": "UniProtKB:Q9HCE6",
  "term_id": "GO:0005737"
}